{
  "gene_name": "Vesicle transport through interaction with t-SNAREs homolog 1B",
  "term_id": "GO:0006896",
  "gene_symbol": "VTI1B",
  "term_label": "Golgi to vacuole transport",
  "gene": "UniProtKB:Q9UEU0"
}